complement component C4b binding [GO:0001855] (molecular function) Relationships: is a type of GO:0001846; is a type of complement binding [GO:0001848] Sources: GOC:add, ISBN:0781735149 Definition: Binding to a C4b product of the classical complement cascade.